{
  "term_id": "GO:0000981",
  "term_label": "DNA-binding transcription factor activity, RNA polymerase II-specific",
  "gene_symbol": "HOXD11",
  "gene_name": "Homeobox protein Hox-D11",
  "gene": "UniProtKB:P31277"
}